{
  "gene_symbol": "C19orf67",
  "gene": "UniProtKB:A6NJJ6",
  "term_label": "Unknown cellular component",
  "gene_name": "UPF0575 protein C19orf67",
  "term_id": "UNKNOWN:0003"
}